{
  "gene_name": "Transcription factor HIVEP2",
  "term_label": "regulation of transcription by RNA polymerase II",
  "term_id": "GO:0006357",
  "gene_symbol": "HIVEP2",
  "gene": "UniProtKB:P31629"
}